{
  "gene_symbol": "MYOM2",
  "term_id": "GO:0045214",
  "term_label": "sarcomere organization",
  "gene": "UniProtKB:P54296",
  "gene_name": "Myomesin-2"
}